symbiont-mediated perturbation of host inflammatory response [GO:0052032] (biological process) Sources: GOC:mtg_pamgo_17jul06 Subtypes: symbiont-mediated suppression of host inflammatory response [GO:0052036] Definition: A process in which a symbiont alters or subverts the normal execution of the  inflammatory response of the host organism; the inflammatory response is the immediate defensive reaction (by vertebrate tissue) to infection or injury caused by chemical or physical agents. The host is defined as the larger of the organisms involved in a symbiotic interaction. Also known as: modulation by organism of inflammatory response of other organism involved in symbiotic interaction, modulation by symbiont of host inflammatory response, perturbation by symbiont of host inflammatory response Relationships: is a type of symbiont-mediated perturbation of host innate immune response [GO:0052167]